pyruvate decarboxylation to acetyl-CoA [GO:0006086] (biological process) Regulation: regulated by regulation of pyruvate decarboxylation to acetyl-CoA [GO:0010510]; RO_0002213 by positive regulation of pyruvate decarboxylation to acetyl-CoA [GO:0140176]; negatively regulated by GO:0160218 Definition: The chemical reactions and pathways resulting in the formation of acetyl-CoA from pyruvate.  In most organisms, this pathway links glycolysis to the TCA cycle, by a series of three reactions carried out by a multisubunit complex called the 'pyruvate dehydrogenase complex', even though pyruvate dehydrogenase activity describes only one of those reactions. The combination of the three reactions can be summarized as: pyruvate + coenzyme A + NAD+ -> acetyl-CoA + CO2 + NADH. Relationships: is a type of acetyl-CoA biosynthetic process [GO:0006085]; is a type of GO:0006090; BFO_0000050 GO:0009060; has part GO:0004148; BFO_0000051 GO:0004739; has part GO:0004742 Sources: MetaCyc:PYRUVDEHYD-PWY Also known as: acetyl-CoA anabolism from pyruvate, acetyl-CoA biosynthetic process from pyruvate, acetyl-CoA formation from pyruvate, acetyl-CoA synthesis from pyruvate, oxidative decarboxylation of pyruvate, pyruvate dehydrogenase pathway, pyruvate decarboxylation